positive regulation of interleukin-8 production [GO:0032757] (biological process) Also known as: positive regulation of IL-8 production, up regulation of interleukin-8 production, up-regulation of interleukin-8 production, upregulation of interleukin-8 production, activation of interleukin-8 production, positive regulation of interleukin-8 biosynthetic process, positive regulation of interleukin-8 secretion, stimulation of interleukin-8 production Relationships: is a type of positive regulation of cytokine production [GO:0001819]; is a type of regulation of interleukin-8 production [GO:0032677]; positively regulates interleukin-8 production [GO:0032637] Definition: Any process that activates or increases the frequency, rate, or extent of interleukin-8 production. Sources: GOC:mah